{
  "term_id": "UNKNOWN:0003",
  "term_label": "Unknown cellular component",
  "gene": "UniProtKB:Q6DD88",
  "gene_symbol": "ATL3",
  "gene_name": "Atlastin-3"
}